{
  "gene_name": "Enkurin",
  "gene": "UniProtKB:Q8TC29",
  "term_label": "axonemal microtubule",
  "gene_symbol": "ENKUR",
  "term_id": "GO:0005879"
}